{
  "term_label": "membrane",
  "gene": "UniProtKB:Q9UF11",
  "term_id": "GO:0016020",
  "gene_symbol": "PLEKHB1",
  "gene_name": "Pleckstrin homology domain-containing family B member 1"
}